{
  "gene": "UniProtKB:Q15762",
  "term_id": "GO:0050839",
  "gene_symbol": "CD226",
  "gene_name": "CD226 antigen",
  "term_label": "cell adhesion molecule binding"
}